positive regulation of apoptotic process in bone marrow cell [GO:0120132] (biological process) Relationships: is a type of positive regulation of apoptotic process [GO:0043065]; is a type of GO:0071865; positively regulates GO:0071839 References: PMID:27908889 Sources: GOC:BHF, GOC:BHF_miRNA, GOC:rph Also known as: positive regulation of apoptotic process in bone marrow, positive regulation of bone marrow cell apoptosis, positive regulation of bone marrow cell programmed cell death by apoptosis, positive regulation of killing of bone marrow cells, positive regulation of programmed cell death of bone marrow cells by apoptosis, positive regulation of programmed cell death, bone marrow cells, up regulation of apoptosis in bone marrow, up-regulation of apoptosis in bone marrow, upregulation of apoptosis in bone marrow, activation of apoptosis in bone marrow, positive regulation of apoptosis in bone marrow Definition: Any process that activates or increases the frequency, rate or extent of cell death by apoptotic process in the bone marrow.